galactotriose transport [GO:2001093] (biological process) Relationships: is a type of trisaccharide transport [GO:2001088] Definition: The directed movement of a galactotrioseacetate into, out of or within a cell, or between cells, by means of some agent such as a transporter or pore. Sources: GOC:mengo_curators Regulation: regulated by regulation of galactotriose transport [GO:1900291]; negatively regulated by negative regulation of galactotriose transport [GO:1900292]; positively regulated by positive regulation of galactotriose transport [GO:1900293]